{
  "term_label": "Unknown molecular function",
  "gene": "UniProtKB:Q9NSQ0",
  "gene_symbol": "RRP7BP",
  "term_id": "UNKNOWN:0001",
  "gene_name": "Putative ribosomal RNA-processing protein 7 homolog B"
}